{
  "term_id": "UNKNOWN:0003",
  "gene_name": "Coiled-coil domain-containing protein 166",
  "gene_symbol": "CCDC166",
  "term_label": "Unknown cellular component",
  "gene": "UniProtKB:P0CW27"
}